{
  "term_label": "cell migration",
  "gene_name": "Syndecan-3",
  "gene_symbol": "SDC3",
  "gene": "UniProtKB:O75056",
  "term_id": "GO:0016477"
}